{
  "term_id": "GO:0016192",
  "gene_name": "Ras-related protein Rab-4A",
  "term_label": "vesicle-mediated transport",
  "gene_symbol": "RAB4A",
  "gene": "UniProtKB:P20338"
}